{
  "term_label": "presynaptic membrane",
  "gene": "UniProtKB:Q96PR1",
  "gene_symbol": "KCNC2",
  "gene_name": "Potassium voltage-gated channel subfamily C member 2",
  "term_id": "GO:0042734"
}